6-carboxymethyl-5-methyl-4-hydroxypyridin-2-ol 3-C-methyltransferase activity [GO:0160302] (molecular function) References: PMID:27391308 Definition: Catalysis of the reaction: 6-carboxymethyl-5-methyl-4-hydroxypyridin-2-ol + S-adenosyl-L-methionine = 6-carboxymethyl-3,5-dimethyl-4-hydroxypyridin-2-ol + S-adenosyl-L-homocysteine + H+. Relationships: is a type of methyltransferase activity [GO:0008168]